{
  "gene_symbol": "UBE2B",
  "gene_name": "Ubiquitin-conjugating enzyme E2 B",
  "term_id": "GO:0006281",
  "term_label": "DNA repair",
  "gene": "UniProtKB:P63146"
}